{
  "gene": "UniProtKB:Q7Z5L2",
  "gene_name": "Coiled-coil domain-containing protein R3HCC1L",
  "term_id": "UNKNOWN:0002",
  "gene_symbol": "R3HCC1L",
  "term_label": "Unknown biological process"
}